paraherquonin biosynthetic process [GO:0140874] (biological process) Definition: The chemical reactions and pathways resulting in the formation of paraherquonin, a meroterpenoid with a unique, highly congested hexacyclic molecular architecture. References: PMID:27602587 Also known as: paraherquonin anabolism, paraherquonin biosynthesis, paraherquonin formation, paraherquonin synthesis Relationships: is a type of terpenoid biosynthetic process [GO:0016114]; is a type of ketone biosynthetic process [GO:0042181]; is a type of GO:1901336; is a type of tertiary alcohol biosynthetic process [GO:1902645]